{
  "term_label": "Unknown molecular function",
  "gene_name": "Leucine-rich repeat transmembrane neuronal protein 2",
  "term_id": "UNKNOWN:0001",
  "gene_symbol": "LRRTM2",
  "gene": "UniProtKB:O43300"
}